{
  "term_label": "Unknown biological process",
  "gene_name": "Protein O-glucosyltransferase 2",
  "gene_symbol": "POGLUT2",
  "term_id": "UNKNOWN:0002",
  "gene": "UniProtKB:Q6UW63"
}